{
  "gene_name": "Choline kinase alpha",
  "gene": "UniProtKB:P35790",
  "term_id": "GO:0004103",
  "term_label": "choline kinase activity",
  "gene_symbol": "CHKA"
}